{
  "term_label": "calcium/calmodulin-dependent protein kinase activity",
  "term_id": "GO:0004683",
  "gene_symbol": "MAPKAPK3",
  "gene_name": "MAP kinase-activated protein kinase 3",
  "gene": "UniProtKB:Q16644"
}